{
  "gene_symbol": "REP15",
  "term_id": "GO:0055037",
  "term_label": "recycling endosome",
  "gene_name": "Rab15 effector protein",
  "gene": "UniProtKB:Q6BDI9"
}